{
  "term_id": "GO:0015020",
  "gene": "UniProtKB:P16662",
  "term_label": "glucuronosyltransferase activity",
  "gene_name": "UDP-glucuronosyltransferase 2B7",
  "gene_symbol": "UGT2B7"
}